{
  "term_label": "Unknown biological process",
  "term_id": "UNKNOWN:0002",
  "gene": "UniProtKB:Q9NZB2",
  "gene_name": "Constitutive coactivator of PPAR-gamma-like protein 1",
  "gene_symbol": "FAM120A"
}